{
  "term_id": "UNKNOWN:0003",
  "term_label": "Unknown cellular component",
  "gene_symbol": "TIA1",
  "gene_name": "Cytotoxic granule associated RNA binding protein TIA1",
  "gene": "UniProtKB:P31483"
}